{
  "term_label": "adherens junction organization",
  "gene_name": "Cadherin-3",
  "gene_symbol": "CDH3",
  "term_id": "GO:0034332",
  "gene": "UniProtKB:P22223"
}